positive regulation of toll-like receptor 8 signaling pathway [GO:0034161] (biological process) Also known as: positive regulation of TLR8 signaling pathway, positive regulation of toll-like receptor 8 signalling pathway Definition: Any process that activates or increases the frequency, rate, or extent of toll-like receptor 8 signaling pathway. Relationships: is a type of regulation of toll-like receptor 8 signaling pathway [GO:0034159]; is a type of positive regulation of pattern recognition receptor signaling pathway [GO:0062208]; is a type of positive regulation of intracellular signal transduction [GO:1902533]; positively regulates toll-like receptor 8 signaling pathway [GO:0034158] References: PMID:16551253, PMID:17328678 Sources: GOC:add